protein-transporting ATPase activity [GO:0015450] (molecular function) Subtypes: protein-exporting ATPase activity [GO:0008564], mitochondrial protein-transporting ATPase activity [GO:0008566], GO:0015462, chloroplast protein-transporting ATPase activity [GO:0016464] Relationships: is_a protein transmembrane transporter activity [GO:0008320]; is a type of ATPase-coupled transmembrane transporter activity [GO:0042626] Also known as: protein translocase activity, P-P-bond-hydrolysis-driven protein transmembrane transporter activity Sources: GOC:mtg_transport, ISBN:0815340729 Definition: Primary active carrier-mediated transport of a protein across a membrane, driven by the hydrolysis of the diphosphate bond of inorganic pyrophosphate, ATP, or another nucleoside triphosphate. The transport protein may or may not be transiently phosphorylated, but the substrate is not phosphorylated.